N-acyl-D-glutamate deacylase activity [GO:0047421] (molecular function) Relationships: is a type of hydrolase activity, acting on carbon-nitrogen (but not peptide) bonds, in linear amides [GO:0016811] Sources: EC:3.5.1.82, RHEA:12833 Definition: Catalysis of the reaction: N-acyl-D-glutamate + H2O = D-glutamate + a carboxylate. Also known as: N-acyl-D-glutamate amidohydrolase activity